{
  "gene_symbol": "SGCE",
  "gene_name": "Epsilon-sarcoglycan",
  "term_label": "Unknown molecular function",
  "term_id": "UNKNOWN:0001",
  "gene": "UniProtKB:O43556"
}